{
  "gene": "UniProtKB:P55160",
  "gene_symbol": "NCKAP1L",
  "term_id": "GO:0030031",
  "term_label": "cell projection assembly",
  "gene_name": "Nck-associated protein 1-like"
}